progesterone monooxygenase activity [GO:0050214] (molecular function) Definition: Catalysis of the reaction: AH2 + O2 + progesterone = A + H2O + testosterone acetate. Also known as: progesterone hydroxylase activity, progesterone,hydrogen-donor:oxygen oxidoreductase (hydroxylating) Subtypes: progesterone 11-alpha-monooxygenase activity [GO:0050212] Relationships: is a type of steroid hydroxylase activity [GO:0008395]; is_a oxidoreductase activity, acting on paired donors, with incorporation or reduction of molecular oxygen [GO:0016705] References: PMID:5950688 Sources: RHEA:11984